detection of oomycetes [GO:0002231] (biological process) References: PMID:15922649 Sources: GOC:add Definition: The series of events in which a stimulus from an oomycetes is received and converted into a molecular signal. Relationships: is a type of response to oomycetes [GO:0002239]; is a type of detection of other organism [GO:0098543]